{
  "term_id": "GO:0140658",
  "gene_name": "Chromodomain-helicase-DNA-binding protein 3",
  "term_label": "ATP-dependent chromatin remodeler activity",
  "gene": "UniProtKB:Q12873",
  "gene_symbol": "CHD3"
}